TRAMP complex [GO:0031499] (CC) Definition: A multiprotein complex having distributive polyadenylation activity of a variety of RNA substrates including hypomodified and incorrectly folded tRNAs, pre-snRNAs, pre-snoRNAs, incorrectly spliced or processed pre-mRNAs, cryptic unstable transcripts (CUTs), pre-rRNAs and rRNA fragments released as part of rRNA processing. In S. cerevisiae, the complex consists of either Pap2 (also known as Trf4) or Trf5, Air1 or Air2, and Mtr4, and is involved in RNA 3'-end processing and in RNA surveillance and quality control. Relationships: is a type of nuclear protein-containing complex [GO:0140513] References: PMID:15173578, PMID:15828860, PMID:15935758, PMID:15935759, PMID:16373491, PMID:16374505, PMID:16431988, PMID:16973437, PMID:17410208, PMID:17652137 Also known as: TRAMP4 complex, TRAMP5 complex, Trf4 complex, Trf4 poly(A) polymerase complex, Trf4p-Air2p-Mtr4p polyadenylation complex